regulation of juvenile hormone biosynthetic process [GO:0007557] (BP) Sources: GOC:go_curators Also known as: regulation of juvenile hormone anabolism, regulation of juvenile hormone biosynthesis, regulation of juvenile hormone formation, regulation of juvenile hormone synthesis Definition: Any process that modulates the frequency, rate or extent of the chemical reactions and pathways resulting in the formation of juvenile hormone. Subtypes: negative regulation of juvenile hormone biosynthetic process [GO:0045968], positive regulation of juvenile hormone biosynthetic process [GO:0045969] Relationships: is a type of regulation of isoprenoid metabolic process [GO:0019747]; is a type of regulation of hormone biosynthetic process [GO:0046885]; is a type of regulation of lipid biosynthetic process [GO:0046890]; regulates juvenile hormone biosynthetic process [GO:0006718]